{
  "gene": "UniProtKB:Q5T953",
  "gene_name": "Immediate early response gene 5-like protein",
  "term_label": "Unknown molecular function",
  "term_id": "UNKNOWN:0001",
  "gene_symbol": "IER5L"
}